{
  "gene_name": "Interleukin-1 receptor-associated kinase-like 2",
  "term_id": "GO:0035556",
  "gene_symbol": "IRAK2",
  "term_label": "intracellular signal transduction",
  "gene": "UniProtKB:O43187"
}